{
  "term_label": "Unknown cellular component",
  "gene": "UniProtKB:A8MTW9",
  "gene_symbol": "A8MTW9",
  "term_id": "UNKNOWN:0003",
  "gene_name": "Putative uncharacterized protein ENSP00000380674"
}